{
  "term_label": "plasma membrane",
  "gene_symbol": "ITPR1",
  "gene": "UniProtKB:Q14643",
  "gene_name": "Inositol 1,4,5-trisphosphate receptor type 1",
  "term_id": "GO:0005886"
}